tRNA methyltransferase activator activity [GO:0141106] (molecular function) Definition: Binds to and increases the activity of a methyltransferase. Relationships: is a type of GO:0008047; is a type of GO:0141107; positively regulates methyltransferase activity [GO:0008168] Sources: GOC:curators